{
  "gene": "UniProtKB:Q3KP66",
  "term_label": "adherens junction maintenance",
  "term_id": "GO:0034334",
  "gene_name": "Innate immunity activator protein",
  "gene_symbol": "INAVA"
}